nuclear RNA export factor complex [GO:0042272] (cellular component) Also known as: Mex67-Mtr2 complex, NXF1-NXT1 complex, TAP-p15 complex Relationships: is a type of GO:0140513 Definition: A protein complex that contains two proteins (know in several organisms, including Drosophila, as NXF1 and NXF2) and is required for the export of the majority of mRNAs from the nucleus to the cytoplasm; localized in the nucleoplasm and at both the nucleoplasmic and cytoplasmic faces of the nuclear pore complex; shuttles between the nucleus and the cytoplasm. References: PMID:11780633